{
  "term_id": "UNKNOWN:0002",
  "gene_name": "GTPase IMAP family member 2",
  "gene": "UniProtKB:Q9UG22",
  "term_label": "Unknown biological process",
  "gene_symbol": "GIMAP2"
}